positive regulation of dentin-containing tooth bud formation by mesenchymal-epithelial signaling [GO:0060640] (biological process) Also known as: positive regulation of dentine-containing tooth bud formation by mesenchymal-epithelial signalling, positive regulation of dentine-containing tooth bud formation by mesenchymal-epithelial signaling Relationships: is a type of GO:0042488; is a type of mesenchymal-epithelial cell signaling [GO:0060638] Definition: Any process that initiates the formation of a tooth bud by the secretion of a signal from a mesenchymal cell and its reception and subsequent change in the identity of an epithelial cell of the tooth bud. Sources: GOC:dph